{
  "gene_name": "Phospholipid-transporting ATPase ABCA7",
  "term_id": "UNKNOWN:0003",
  "gene": "UniProtKB:Q8IZY2",
  "term_label": "Unknown cellular component",
  "gene_symbol": "ABCA7"
}